{
  "gene_name": "Erythropoietin receptor",
  "term_label": "erythropoietin receptor activity",
  "term_id": "GO:0004900",
  "gene": "UniProtKB:P19235",
  "gene_symbol": "EPOR"
}